{
  "term_label": "Unknown molecular function",
  "gene_name": "Serine incorporator 4",
  "gene": "UniProtKB:A6NH21",
  "term_id": "UNKNOWN:0001",
  "gene_symbol": "SERINC4"
}